mitochondrial chromosome packaging [GO:0090139] (biological process) Relationships: is a type of GO:0051276; occurs in mitochondrion [GO:0005739] Sources: GOC:ascb_2009, GOC:dph, GOC:tb Also known as: mitochondrial DNA packaging Definition: A process in which mitochondrial chromosomal DNA and associated proteins organize into a compact, orderly structure.